{
  "gene_name": "Caspase-3",
  "gene_symbol": "CASP3",
  "term_id": "GO:0005737",
  "term_label": "cytoplasm",
  "gene": "UniProtKB:P42574"
}